{
  "gene_name": "5-hydroxytryptamine receptor 4",
  "term_id": "GO:0030425",
  "term_label": "dendrite",
  "gene": "UniProtKB:Q13639",
  "gene_symbol": "HTR4"
}